{
  "term_id": "GO:0031201",
  "gene": "UniProtKB:Q9P2W9",
  "term_label": "SNARE complex",
  "gene_symbol": "STX18",
  "gene_name": "Syntaxin-18"
}